{
  "gene_symbol": "PSME2",
  "term_id": "GO:2000045",
  "gene_name": "Proteasome activator complex subunit 2",
  "gene": "UniProtKB:Q9UL46",
  "term_label": "regulation of G1/S transition of mitotic cell cycle"
}